{
  "gene_name": "Thrombomodulin",
  "term_id": "UNKNOWN:0002",
  "term_label": "Unknown biological process",
  "gene": "UniProtKB:P07204",
  "gene_symbol": "THBD"
}